{
  "gene_name": "Zinc finger protein-like 1",
  "gene": "UniProtKB:O95159",
  "gene_symbol": "ZFPL1",
  "term_label": "Unknown molecular function",
  "term_id": "UNKNOWN:0001"
}